benzylpenicillin metabolic process [GO:1901086] (biological process) Relationships: is a type of GO:0042316 Also known as: benzylpenicillin metabolism, penicillin G metabolism Sources: GOC:TermGenie, GOC:yaf, UniPathway:UPA00149 Subtypes: GO:1901087, GO:1901088 Definition: The chemical reactions and pathways involving benzylpenicillin.